{
  "term_id": "UNKNOWN:0001",
  "gene_symbol": "RP1L1",
  "gene": "UniProtKB:Q8IWN7",
  "term_label": "Unknown molecular function",
  "gene_name": "Retinitis pigmentosa 1-like 1 protein"
}